{
  "gene_name": "Leucine-rich repeat and immunoglobulin-like domain-containing nogo receptor-interacting protein 4",
  "gene": "UniProtKB:Q6UY18",
  "term_id": "UNKNOWN:0002",
  "gene_symbol": "LINGO4",
  "term_label": "Unknown biological process"
}